{
  "term_id": "GO:0000981",
  "term_label": "DNA-binding transcription factor activity, RNA polymerase II-specific",
  "gene_symbol": "ZNF324B",
  "gene_name": "Zinc finger protein 324B",
  "gene": "UniProtKB:Q6AW86"
}